{
  "term_label": "Unknown molecular function",
  "term_id": "UNKNOWN:0001",
  "gene": "UniProtKB:Q96QK8",
  "gene_symbol": "SMIM14",
  "gene_name": "Small integral membrane protein 14"
}